{
  "gene_symbol": "THAP5",
  "term_id": "UNKNOWN:0002",
  "gene": "UniProtKB:Q7Z6K1",
  "gene_name": "THAP domain-containing protein 5",
  "term_label": "Unknown biological process"
}